metal ion sequestering activity [GO:0140487] (molecular function) References: PMID:12050156 Subtypes: calcium ion sequestering activity [GO:0140314], iron ion sequestering activity [GO:0140315], zinc ion sequestering activity [GO:0140486] Definition: Binding to a metal ion to prevent it from interacting with other partners or to inhibit its localization to the area of the cell or complex where it is active. Relationships: is_a GO:0140313; has part metal ion binding [GO:0046872]